{
  "gene_name": "Immunoglobulin heavy variable 4-4",
  "term_label": "antigen binding",
  "gene": "UniProtKB:A0A075B6R2",
  "gene_symbol": "IGHV4-4",
  "term_id": "GO:0003823"
}